{
  "term_id": "GO:0006887",
  "gene": "UniProtKB:Q16623",
  "gene_symbol": "STX1A",
  "term_label": "exocytosis",
  "gene_name": "Syntaxin-1A"
}